{
  "term_id": "GO:0005516",
  "gene_name": "IQ domain-containing protein F1",
  "term_label": "calmodulin binding",
  "gene": "UniProtKB:Q8N6M8",
  "gene_symbol": "IQCF1"
}